{
  "gene": "UniProtKB:Q5MY95",
  "gene_symbol": "ENTPD8",
  "term_label": "UDP phosphatase activity",
  "term_id": "GO:0045134",
  "gene_name": "Ectonucleoside triphosphate diphosphohydrolase 8"
}